EGF-domain serine glucosyltransferase activity [GO:0140561] (molecular function) Definition: Catalysis of the reaction: UDP-alpha-D-glucose + [protein with EGF-like domain]-L-serine = UDP + [protein with EGF-like domain]-3-O-(beta-D-glucosyl)-L-serine. Relationships: is a type of UDP-glucosyltransferase activity [GO:0035251] Sources: RHEA:58116